peroxidase inhibitor activity [GO:0036479] (molecular function) Definition: Binds to and stops, prevents or reduces the activity of peroxidase. Relationships: is a type of enzyme inhibitor activity [GO:0004857]; negatively regulates GO:0004601 Sources: GOC:PARL, GOC:bf Note: GO:0036479 is reserved for cases when the inhibitor directly interacts with the peroxidase. When inhibition of peroxidase activity is achieved without enzyme binding, or when the mechanism of regulation is unknown, instead annotate to 'negative regulation of peroxidase activity ; GO:2000469'.